siderophore transmembrane transport [GO:0044718] (biological process) Definition: The directed movement of siderophores, low molecular weight Fe(III)-chelating substances, from one side of a membrane to the other, by means of some agent such as a transporter or pore. Relationships: is a type of GO:0015891 Also known as: siderophore membrane transport Sources: GOC:jl Note: Note that this term is not intended for use in annotating lateral movement within membranes.